{
  "gene_name": "Potassium voltage-gated channel subfamily A member 1",
  "gene": "UniProtKB:Q09470",
  "gene_symbol": "KCNA1",
  "term_label": "potassium ion transmembrane transport",
  "term_id": "GO:0071805"
}